{
  "gene_symbol": "PRMT6",
  "term_id": "GO:0006355",
  "term_label": "regulation of DNA-templated transcription",
  "gene": "UniProtKB:Q96LA8",
  "gene_name": "Protein arginine N-methyltransferase 6"
}